{
  "term_id": "UNKNOWN:0001",
  "gene": "UniProtKB:A4D1E1",
  "term_label": "Unknown molecular function",
  "gene_symbol": "ZNF804B",
  "gene_name": "Zinc finger protein 804B"
}